{
  "term_label": "Unknown cellular component",
  "term_id": "UNKNOWN:0003",
  "gene_name": "Transforming growth factor beta receptor type 3",
  "gene_symbol": "TGFBR3",
  "gene": "UniProtKB:Q03167"
}